{
  "gene_name": "Pleckstrin homology-like domain family A member 3",
  "gene_symbol": "PHLDA3",
  "term_label": "plasma membrane",
  "gene": "UniProtKB:Q9Y5J5",
  "term_id": "GO:0005886"
}